{
  "gene_name": "Olfactory receptor 2J2",
  "gene": "UniProtKB:O76002",
  "gene_symbol": "OR2J2",
  "term_id": "GO:0004984",
  "term_label": "olfactory receptor activity"
}